{
  "gene_symbol": "ABCC11",
  "term_label": "plasma membrane",
  "gene": "UniProtKB:Q96J66",
  "gene_name": "ATP-binding cassette sub-family C member 11",
  "term_id": "GO:0005886"
}